positive regulation of vesicle docking [GO:0106022] (biological process) Definition: Any process that activates or increases the frequency, rate or extent of vesicle docking. References: PMID:22810233 Also known as: positive regulation of vesicle to membrane docking Relationships: is a type of positive regulation of cellular process [GO:0048522]; is_a GO:0106020; positively regulates vesicle docking [GO:0048278]